{
  "term_id": "GO:0034205",
  "gene": "UniProtKB:P49768",
  "gene_symbol": "PSEN1",
  "term_label": "amyloid-beta formation",
  "gene_name": "Presenilin-1"
}